(5alpha)-campestan-3-one hydroxylase activity [GO:0102679] (molecular function) Definition: Catalysis of the reaction: H+ + (5alpha)-campestan-3-one + O2 + NADPH = (5alpha,22S,24R)-22-hydroxyergostan-3-one + H2O + NADP. References: PMID:10377996 Sources: GOC:pz Relationships: is a type of oxidoreductase activity, acting on paired donors, with incorporation or reduction of molecular oxygen, NAD(P)H as one donor, and incorporation of one atom of oxygen [GO:0016709]